{
  "gene_name": "Rho GTPase-activating protein SYDE2",
  "gene": "UniProtKB:Q5VT97",
  "term_label": "GTPase activator activity",
  "gene_symbol": "SYDE2",
  "term_id": "GO:0005096"
}